cellular response to prostaglandin D stimulus [GO:0071799] (biological process) Definition: Any process that results in a change in state or activity of a cell (in terms of movement, secretion, enzyme production, gene expression, etc.) as a result of a prostagladin D stimulus. Sources: GOC:sl Relationships: is a type of cellular response to prostaglandin stimulus [GO:0071379]; is a type of GO:0071798; is a type of cellular response to alcohol [GO:0097306]; is a type of cellular response to ketone [GO:1901655]